purine ribonucleotide transport [GO:0015868] (biological process) Relationships: is a type of GO:0015865; is a type of carbohydrate derivative transport [GO:1901264] Subtypes: ADP transport [GO:0015866], ATP transport [GO:0015867], 3'-phosphoadenosine 5'-phosphosulfate transport [GO:0046963], cAMP transport [GO:0070730], GO:0070731, adenosine 3',5'-bisphosphate transmembrane transport [GO:0071106], AMP transport [GO:0080121], cyclic-GMP-AMP transmembrane import across plasma membrane [GO:0140361], 5'-adenylyl sulfate transmembrane transport [GO:1902558] Definition: The directed movement of a purine ribonucleotide, any compound consisting of a purine ribonucleoside (a purine organic base attached to a ribose sugar) esterified with (ortho)phosphate, into, out of or within a cell. Sources: GOC:ai